{
  "gene": "UniProtKB:Q9H4S2",
  "term_id": "GO:0000978",
  "term_label": "RNA polymerase II cis-regulatory region sequence-specific DNA binding",
  "gene_symbol": "GSX1",
  "gene_name": "GS homeobox 1"
}